{
  "term_id": "GO:1990817",
  "gene": "UniProtKB:Q9NVV4",
  "term_label": "poly(A) RNA polymerase activity",
  "gene_symbol": "MTPAP",
  "gene_name": "Poly(A) RNA polymerase, mitochondrial"
}